{
  "gene_name": "1-phosphatidylinositol 4,5-bisphosphate phosphodiesterase gamma-1",
  "term_id": "GO:0010634",
  "gene_symbol": "PLCG1",
  "gene": "UniProtKB:P19174",
  "term_label": "positive regulation of epithelial cell migration"
}